oligosaccharide transporting porin activity [GO:0015478] (molecular function) Relationships: is a type of oligosaccharide transmembrane transporter activity [GO:0015157]; is a type of porin activity [GO:0015288] Definition: Enables the transfer of oligosaccharide, sized less than 1000 Da, from one side of a membrane to the other. The transmembrane portions of porins consist exclusively of beta-strands which form a beta-barrel. They are found in the outer membranes of Gram-negative bacteria, mitochondria, plastids and possibly acid-fast Gram-positive bacteria. Also known as: raffinose porin Sources: GOC:mtg_transport